{
  "term_label": "Unknown molecular function",
  "gene": "UniProtKB:Q1XH10",
  "gene_name": "SKI_DACH domain-containing protein 1",
  "term_id": "UNKNOWN:0001",
  "gene_symbol": "SKIDA1"
}